regulation of glycine secretion, neurotransmission [GO:1904624] (biological process) Relationships: is a type of GO:0032890; is a type of regulation of neurotransmitter secretion [GO:0046928]; is_a GO:0051955; is a type of regulation of synaptic transmission, glycinergic [GO:0060092]; regulates glycine secretion, neurotransmission [GO:0061537] Definition: Any process that modulates the frequency, rate or extent of glycine secretion, neurotransmission. Subtypes: negative regulation of glycine secretion, neurotransmission [GO:1904625], positive regulation of glycine secretion, neurotransmission [GO:1904626] References: PMID:22988142 Sources: GOC:TermGenie, GO_REF:0000058